protein C-linked glycosylation [GO:0018103] (biological process) Relationships: is a type of glycoprotein biosynthetic process [GO:0009101] Also known as: protein amino acid C-linked glycosylation References: PMID:35536965, PMID:7947762 Definition: A protein glycosylation process in which a carbohydrate or carbohydrate derivative unit is added to a protein via a C atom.